{
  "term_id": "UNKNOWN:0003",
  "gene_symbol": "OR8G3",
  "gene": "UniProtKB:P0DMU2",
  "term_label": "Unknown cellular component",
  "gene_name": "Putative olfactory receptor 8G3 pseudogene"
}